{
  "gene_symbol": "IL12A",
  "term_id": "GO:0005615",
  "gene": "UniProtKB:P29459",
  "gene_name": "Interleukin-12 subunit alpha",
  "term_label": "extracellular space"
}